{
  "gene_symbol": "GSDMD",
  "term_id": "GO:0042742",
  "gene": "UniProtKB:P57764",
  "gene_name": "Gasdermin-D",
  "term_label": "defense response to bacterium"
}